leukocyte chemotaxis involved in inflammatory response [GO:0002232] (biological process) Also known as: immune cell chemotaxis during inflammatory response, leucocyte chemotaxis during inflammatory response, leukocyte chemotaxis during inflammatory response Definition: The movement of an immune cell in response to an external stimulus contributing to an inflammatory response. Sources: GOC:add, ISBN:0781735149 Relationships: is a type of leukocyte migration involved in inflammatory response [GO:0002523]; is a type of leukocyte chemotaxis [GO:0030595]